{
  "gene_symbol": "RPGR",
  "term_label": "ubiquitin-dependent protein catabolic process",
  "term_id": "GO:0006511",
  "gene_name": "X-linked retinitis pigmentosa GTPase regulator",
  "gene": "UniProtKB:Q92834"
}